{
  "gene": "UniProtKB:Q9HBH1",
  "term_id": "GO:0005739",
  "gene_symbol": "PDF",
  "term_label": "mitochondrion",
  "gene_name": "Peptide deformylase, mitochondrial"
}